{
  "term_id": "GO:0042632",
  "gene_name": "Group XIIB secretory phospholipase A2-like protein",
  "gene": "UniProtKB:Q9BX93",
  "term_label": "cholesterol homeostasis",
  "gene_symbol": "PLA2G12B"
}